{
  "term_label": "heterochromatin formation",
  "term_id": "GO:0031507",
  "gene_name": "Histone H3.3C",
  "gene_symbol": "H3-5",
  "gene": "UniProtKB:Q6NXT2"
}